{
  "gene_symbol": "EPO",
  "term_id": "GO:0005615",
  "term_label": "extracellular space",
  "gene": "UniProtKB:P01588",
  "gene_name": "Erythropoietin"
}